{
  "term_id": "UNKNOWN:0001",
  "gene_name": "IQ motif and ankyrin repeat domain-containing protein 1",
  "gene_symbol": "IQANK1",
  "term_label": "Unknown molecular function",
  "gene": "UniProtKB:A8MXQ7"
}